{
  "gene": "UniProtKB:O75936",
  "term_label": "carnitine biosynthetic process",
  "gene_symbol": "BBOX1",
  "term_id": "GO:0045329",
  "gene_name": "Gamma-butyrobetaine dioxygenase"
}